{
  "gene": "UniProtKB:Q9NV58",
  "term_label": "ubiquitin protein ligase activity",
  "gene_symbol": "RNF19A",
  "gene_name": "E3 ubiquitin-protein ligase RNF19A",
  "term_id": "GO:0061630"
}